GDP catabolic process [GO:0046712] (biological process) Also known as: GDP breakdown, GDP catabolism, GDP degradation Definition: The chemical reactions and pathways resulting in the breakdown of GDP, guanosine 5'-diphosphate. Relationships: is a type of purine ribonucleotide catabolic process [GO:0009154]; is a type of purine ribonucleoside diphosphate catabolic process [GO:0009181]; is a type of GDP metabolic process [GO:0046710] Sources: GOC:ai